{
  "term_label": "SUMO transferase activity",
  "term_id": "GO:0019789",
  "gene_name": "RANBP2-like and GRIP domain-containing protein 1",
  "gene_symbol": "RGPD1",
  "gene": "UniProtKB:P0DJD0"
}